{
  "gene": "UniProtKB:Q9BYE0",
  "gene_name": "Transcription factor HES-7",
  "term_id": "GO:0000122",
  "term_label": "negative regulation of transcription by RNA polymerase II",
  "gene_symbol": "HES7"
}